host cell periplasmic space [GO:0044229] (cellular component) Definition: The region between the inner (cytoplasmic) and outer host membrane (Gram-negative Bacteria) or inner host membrane and host cell wall (Fungi). Sources: GOC:rph Relationships: is a type of host cell part [GO:0033643]